{
  "gene_name": "Protein GREB1",
  "gene": "UniProtKB:Q4ZG55",
  "term_label": "Unknown molecular function",
  "gene_symbol": "GREB1",
  "term_id": "UNKNOWN:0001"
}